{
  "gene_name": "Potassium voltage-gated channel subfamily E member 3",
  "term_label": "voltage-gated potassium channel activity involved in ventricular cardiac muscle cell action potential repolarization",
  "gene": "UniProtKB:Q9Y6H6",
  "gene_symbol": "KCNE3",
  "term_id": "GO:1902282"
}